{
  "gene_symbol": "TRAJ39",
  "term_label": "Unknown molecular function",
  "gene": "UniProtKB:A0A075B710",
  "gene_name": "T cell receptor alpha joining 39 (Fragment)",
  "term_id": "UNKNOWN:0001"
}